D-xylose biosynthetic process [GO:0042842] (biological process) Definition: The chemical reactions and pathways resulting in the formation of D-xylose, a naturally occurring plant polysaccharide. Sources: ISBN:0198506732 Also known as: D-xylose anabolism, D-xylose biosynthesis, D-xylose formation, D-xylose synthesis Relationships: is a type of pentose biosynthetic process [GO:0019322]; is a type of D-xylose metabolic process [GO:0042732]